{
  "gene_symbol": "SIX5",
  "term_label": "regulation of transcription by RNA polymerase II",
  "term_id": "GO:0006357",
  "gene": "UniProtKB:Q8N196",
  "gene_name": "Homeobox protein SIX5"
}